{
  "gene": "UniProtKB:Q9H9G7",
  "gene_symbol": "AGO3",
  "term_label": "pre-miRNA processing",
  "gene_name": "Protein argonaute-3",
  "term_id": "GO:0031054"
}